{
  "term_label": "adenylate cyclase-activating G protein-coupled receptor signaling pathway",
  "gene": "UniProtKB:P34972",
  "term_id": "GO:0007189",
  "gene_name": "Cannabinoid receptor 2",
  "gene_symbol": "CNR2"
}